amino acid:monoatomic cation antiporter activity [GO:0140848] (molecular function) Subtypes: 3-sulfino-L-alanine: proton, glutamate antiporter activity [GO:0000514], L-glutamate:proton antiporter activity [GO:0106421], L-alanine:proton antiporter activity [GO:0140407], glycine:proton antiporter activity [GO:0140799], gamma-aminobutyric acid:proton antiporter activity [GO:0140800], L-glutamine, sodium:proton antiporter activity [GO:0140830], L-asparagine, sodium:proton antiporter activity [GO:0140831], L-histidine, sodium:proton antiporter activity [GO:0140832] Definition: Enables the transfer of a solute or solutes from one side of a membrane to the other according to the reaction: solute(out) + monoatomic cation(in) = solute(in) + monoatomic cation(out). Monoatomic cations include H+, Mg2+, Ca2+, etc. Sources: GOC:curators Relationships: is a type of monoatomic cation transmembrane transporter activity [GO:0008324]; is a type of amino acid transmembrane transporter activity [GO:0015171]; is a type of antiporter activity [GO:0015297]